{
  "gene_symbol": "SMS",
  "gene": "UniProtKB:P52788",
  "term_id": "GO:0016768",
  "term_label": "spermine synthase activity",
  "gene_name": "Spermine synthase"
}